microtubule polymerization [GO:0046785] (biological process) Also known as: microtubule assembly, microtubule formation Regulation: regulated by regulation of microtubule polymerization [GO:0031113]; negatively regulated by GO:0031115; positively regulated by positive regulation of microtubule polymerization [GO:0031116] Definition: The addition of tubulin heterodimers to one or both ends of a microtubule. Relationships: is a type of microtubule polymerization or depolymerization [GO:0031109]; is a type of protein polymerization [GO:0051258]; is a type of GO:0097435; has part microtubule nucleation [GO:0007020] Sources: GOC:ai, GOC:go_curators